{
  "term_label": "very-long-chain enoyl-CoA reductase activity",
  "gene": "UniProtKB:Q5HYJ1",
  "gene_name": "Trans-2,3-enoyl-CoA reductase-like",
  "gene_symbol": "TECRL",
  "term_id": "GO:0102758"
}